{
  "gene": "UniProtKB:Q99687",
  "term_label": "brain development",
  "term_id": "GO:0007420",
  "gene_name": "Homeobox protein Meis3",
  "gene_symbol": "MEIS3"
}